{
  "term_id": "UNKNOWN:0001",
  "gene_symbol": "APCDD1L",
  "gene_name": "Protein APCDD1-like",
  "gene": "UniProtKB:Q8NCL9",
  "term_label": "Unknown molecular function"
}